{
  "gene_symbol": "EIF3E",
  "term_label": "nucleus",
  "gene_name": "Eukaryotic translation initiation factor 3 subunit E",
  "term_id": "GO:0005634",
  "gene": "UniProtKB:P60228"
}